{
  "term_id": "GO:0008333",
  "gene_symbol": "DENND3",
  "gene_name": "DENN domain-containing protein 3",
  "term_label": "endosome to lysosome transport",
  "gene": "UniProtKB:A2RUS2"
}